{
  "gene": "UniProtKB:Q6YHU6",
  "term_id": "GO:0032471",
  "gene_name": "Thyroid adenoma-associated protein",
  "gene_symbol": "THADA",
  "term_label": "negative regulation of endoplasmic reticulum calcium ion concentration"
}